{
  "term_label": "endoplasmic reticulum membrane",
  "gene": "UniProtKB:Q9P0L0",
  "gene_symbol": "VAPA",
  "term_id": "GO:0005789",
  "gene_name": "Vesicle-associated membrane protein-associated protein A"
}